{
  "term_label": "plasma membrane",
  "gene": "UniProtKB:P58743",
  "term_id": "GO:0005886",
  "gene_name": "Prestin",
  "gene_symbol": "SLC26A5"
}